{
  "gene": "UniProtKB:Q5HYI8",
  "gene_symbol": "RABL3",
  "term_id": "GO:0006886",
  "gene_name": "Rab-like protein 3",
  "term_label": "intracellular protein transport"
}